NAD+-protein-C-terminal glycine ADP-ribosyltransferase activity [GO:0140802] (molecular function) Definition: Catalysis of the reaction: [protein]-C-terminal glycine + NAD+ = [protein]-C-terminal O-(ADP-D-ribosyl)-glycine + nicotinamide. References: PMID:28525742 Sources: RHEA:58268 Relationships: is a type of GO:1990404